{
  "term_id": "GO:0003713",
  "gene_name": "Cbp_p300-interacting transactivator 2",
  "gene_symbol": "CITED2",
  "term_label": "transcription coactivator activity",
  "gene": "UniProtKB:Q99967"
}